magnesium chelatase complex [GO:0010007] (cellular component) References: PMID:11842180 Definition: A heterotrimeric enzyme complex composed of three subunits, all of which are required for enzyme activity, which catalyzes the chelation of Mg by proto IX in an ATP-dependent manner. Relationships: is a type of GO:1902494; is part of chloroplast [GO:0009507]